{
  "gene": "UniProtKB:Q9BQ51",
  "term_id": "GO:0071222",
  "gene_name": "Programmed cell death 1 ligand 2",
  "term_label": "cellular response to lipopolysaccharide",
  "gene_symbol": "PDCD1LG2"
}